{
  "gene": "UniProtKB:Q96PP9",
  "gene_name": "Guanylate-binding protein 4",
  "gene_symbol": "GBP4",
  "term_id": "GO:0003924",
  "term_label": "GTPase activity"
}